regulation of establishment of competence for transformation [GO:0045304] (biological process) Definition: Any process that modulates the frequency, rate or extent of the process in which a cell becomes able to take up and incorporate extracellular DNA into its genome. Sources: GOC:mlg Also known as: regulator of establishment of competence for transformation activity Relationships: is a type of GO:0048583; is a type of GO:0050794; regulates establishment of competence for transformation [GO:0030420] Subtypes: negative regulation of establishment of competence for transformation [GO:0045808], positive regulation of establishment of competence for transformation [GO:0045809]